{
  "gene_name": "Coiled-coil domain-containing protein 30",
  "term_label": "Unknown cellular component",
  "gene_symbol": "CCDC30",
  "gene": "UniProtKB:Q5VVM6",
  "term_id": "UNKNOWN:0003"
}